{
  "term_label": "Unknown cellular component",
  "term_id": "UNKNOWN:0003",
  "gene_name": "Ankyrin repeat domain-containing protein 9",
  "gene": "UniProtKB:Q96BM1",
  "gene_symbol": "ANKRD9"
}